type 2C serotonin receptor binding [GO:0031828] (molecular function) Relationships: is_a G protein-coupled serotonin receptor binding [GO:0031821] Definition: Binding to a type 2C serotonin receptor. Sources: GOC:mah, GOC:nln Also known as: 5-hydroxytryptamine 2C receptor binding, type 2C serotonin receptor ligand